{
  "gene_symbol": "GNB1",
  "term_id": "GO:0005737",
  "gene_name": "Guanine nucleotide-binding protein G(I)_G(S)_G(T) subunit beta-1",
  "gene": "UniProtKB:P62873",
  "term_label": "cytoplasm"
}